{
  "term_id": "GO:0015267",
  "term_label": "channel activity",
  "gene_symbol": "BCL2L2",
  "gene": "UniProtKB:Q92843",
  "gene_name": "Bcl-2-like protein 2"
}